response to diphenidol [GO:1904560] (biological process) Definition: Any process that results in a change in state or activity of a cell or an organism (in terms of movement, secretion, enzyme production, gene expression, etc.) as a result of a diphenidol stimulus. Subtypes: cellular response to diphenidol [GO:1904561] Relationships: is a type of response to alcohol [GO:0097305]; is a type of response to nitrogen compound [GO:1901698] References: PMID:25796330 Sources: GOC:TermGenie, GOC:mr, GO_REF:0000071